regulation of nurse cell apoptotic process [GO:0045477] (biological process) Definition: Any process that modulates the frequency, rate or extent of nurse cell apoptotic process. References: PMID:11973306 Sources: GOC:mtg_apoptosis Also known as: regulation of nurse cell apoptosis Relationships: is a type of GO:1904748; is a type of regulation of reproductive process [GO:2000241]; regulates nurse cell apoptotic process [GO:0045476] Subtypes: GO:0045849, positive regulation of nurse cell apoptotic process [GO:0045850]